{
  "gene_name": "Nuclear RNA export factor 2",
  "gene_symbol": "NXF2B",
  "term_id": "GO:0016973",
  "gene": "UniProtKB:Q9GZY0",
  "term_label": "poly(A)+ mRNA export from nucleus"
}